auditory receptor cell fate determination [GO:0042668] (biological process) Sources: GOC:go_curators Definition: The process in which a cell becomes capable of differentiating autonomously into an auditory hair cell regardless of its environment; upon determination, the cell fate cannot be reversed. Also known as: auditory hair cell fate determination Relationships: is a type of GO:0048664; is part of auditory receptor cell fate commitment [GO:0009912]